{
  "gene": "UniProtKB:P35222",
  "term_label": "nuclear receptor binding",
  "gene_name": "Catenin beta-1",
  "term_id": "GO:0016922",
  "gene_symbol": "CTNNB1"
}